light-dependent chlorophyll biosynthetic process [GO:0036067] (biological process) Also known as: light dependent chlorophyll biosynthetic process, light-dependent chlorophyll anabolism, light-dependent chlorophyll biosynthesis, light-dependent chlorophyll formation, light-dependent chlorophyll synthesis References: PMID:12242396 Sources: GOC:yaf Relationships: is a type of chlorophyll biosynthetic process [GO:0015995] Subtypes: GO:0036069 Definition: The chemical reactions and pathways resulting in the formation of chlorophyll, any compound of magnesium complexed in a porphyrin (tetrapyrrole) ring and which functions as a photosynthetic pigment, from less complex precursors, which occur in the presence of light.